{
  "gene_symbol": "CRAT",
  "term_label": "carnitine metabolic process, CoA-linked",
  "gene": "UniProtKB:P43155",
  "gene_name": "Carnitine O-acetyltransferase",
  "term_id": "GO:0019254"
}